{
  "term_id": "GO:0045944",
  "gene_symbol": "KAT2B",
  "term_label": "positive regulation of transcription by RNA polymerase II",
  "gene_name": "Histone acetyltransferase KAT2B",
  "gene": "UniProtKB:Q92831"
}